{
  "term_label": "negative regulation of TORC1 signaling",
  "gene": "UniProtKB:P54646",
  "term_id": "GO:1904262",
  "gene_name": "5'-AMP-activated protein kinase catalytic subunit alpha-2",
  "gene_symbol": "PRKAA2"
}